{
  "gene": "UniProtKB:A0A0U1RR37",
  "term_label": "Unknown cellular component",
  "gene_name": "Uncharacterized protein C1orf232",
  "gene_symbol": "C1orf232",
  "term_id": "UNKNOWN:0003"
}